{
  "gene_symbol": "ICOSLG",
  "term_label": "signaling receptor binding",
  "gene_name": "ICOS ligand",
  "gene": "UniProtKB:O75144",
  "term_id": "GO:0005102"
}